RNA polymerase IV transcription regulator complex [GO:0090577] (cellular component) Relationships: is a type of transcription regulator complex [GO:0005667] Also known as: RNA polymerase IV transcription factor complex Sources: GOC:tb Definition: A transcription factor complex that acts at a regulatory region of a gene transcribed by RNA polymerase IV.